{
  "gene_symbol": "RCC2",
  "gene_name": "Protein RCC2",
  "gene": "UniProtKB:Q9P258",
  "term_id": "UNKNOWN:0003",
  "term_label": "Unknown cellular component"
}